{
  "term_id": "UNKNOWN:0001",
  "gene_symbol": "TDRG1",
  "gene": "UniProtKB:Q3Y452",
  "term_label": "Unknown molecular function",
  "gene_name": "Testis development-related protein 1"
}